codeine O-demethylase activity [GO:0102805] (molecular function) Relationships: is a type of 2-oxoglutarate-dependent dioxygenase activity [GO:0016706] Definition: Catalysis of the reaction: codeine + 2-oxoglutarate + O2 = morphine + formaldehyde + succinate + CO2. Sources: RHEA:27413